dibenzofuran catabolic process [GO:0019340] (biological process) Relationships: is_a dibenzofuran metabolic process [GO:0018893]; is a type of xenobiotic catabolic process [GO:0042178] Also known as: dibenzofuran breakdown, dibenzofuran catabolism, dibenzofuran degradation Definition: The chemical reactions and pathways resulting in the breakdown of dibenzofuran, a substance composed of two benzene rings linked by one ether bond and one carbon-carbon bond. Sources: GOC:ai